histone H3K36 dimethyltransferase activity [GO:0140954] (MF) Definition: Catalysis of the reaction: L-lysyl36-[histone H3] + 2 S-adenosyl-L-methionine = 2 H+ + N6,N6-dimethyl-L-lysyl36-[histone H3] + 2 S-adenosyl-L-homocysteine. This reaction is the successive addition of two methyl groups to the lysine residue at position 36 of histone H3, producing histone H3K36me2. Sources: RHEA:60308 Also known as: histone H3-K36 dimethylation, histone H3K36 dimethylation, histone H3K36 dimethylase activity, histone H3K36 mono/dimethylase activity, histone lysine N-dimethyltransferase activity (H3-K36 specific) Note: Comment: Note that the residue position corresponds to the canonical human H3 histone (UniProtKB:P84243); this residue is conserved across all eukaryotes. Residue 1 is the first residue following removal of the initiating Methionine (Met). Note that each histone is encoded by multiple genes, and sequences may vary across different genes within an organism. Relationships: is a type of histone H3K36 methyltransferase activity [GO:0046975]